cerebellar Purkinje cell layer formation [GO:0021694] (biological process) Definition: The process that gives rise to the cerebellar Purkinje cell layer. This process pertains to the initial formation of a structure from unspecified parts. The Purkinje cell layer lies just underneath the molecular layer of the cerebellar cortex. It contains the neuronal cell bodies of the Purkinje cells that are arranged side by side in a single layer. Candelabrum interneurons are vertically oriented between the Purkinje cells. Purkinje neurons are inhibitory and provide the output of the cerebellar cortex through axons that project into the white matter. Extensive dendritic trees from the Purkinje cells extend upward in a single plane into the molecular layer where they synapse with parallel fibers of granule cells. Sources: GOC:cls, GOC:dgh, GOC:dph, GOC:jid, GO_REF:0000021 Relationships: is a type of anatomical structure formation involved in morphogenesis [GO:0048646]; is part of cerebellar Purkinje cell layer morphogenesis [GO:0021692]; is part of GO:0021697